luciferin monooxygenase activity [GO:0045289] (molecular function) Sources: GOC:bf Also known as: luciferase activity, luciferase monooxygenase activity Relationships: is a type of monooxygenase activity [GO:0004497] Subtypes: Oplophorus-luciferin 2-monooxygenase activity [GO:0033756], Photinus-luciferin 4-monooxygenase (ATP-hydrolyzing) activity [GO:0047077], GO:0047098, Cypridina-luciferin 2-monooxygenase activity [GO:0047712], Renilla-luciferin 2-monooxygenase activity [GO:0050248], Watasenia-luciferin 2-monooxygenase activity [GO:0050397] Definition: Catalysis of the generalized reaction: luciferin + O2 = oxidized luciferin + CO2 + light. There may be additional substrates and reactants involved in the reaction. The reaction results in light emission as luciferin returns to the ground state after enzymatic oxidation.